phospholipid metabolic process [GO:0006644] (biological process) Sources: ISBN:0198506732 Relationships: is a type of lipid metabolic process [GO:0006629]; is a type of GO:0006796; is_a organophosphate metabolic process [GO:0019637] Definition: The chemical reactions and pathways involving phospholipids, any lipid containing phosphoric acid as a mono- or diester. Regulation: regulated by GO:1903725; negatively regulated by GO:1903726; positively regulated by GO:1903727 Also known as: phospholipid metabolism Subtypes: glycerophospholipid metabolic process [GO:0006650], sphinganine-1-phosphate metabolic process [GO:0006668], inositol phosphoceramide metabolic process [GO:0006673], GO:0006684, phospholipid biosynthetic process [GO:0008654], phospholipid catabolic process [GO:0009395], geranyl diphosphate metabolic process [GO:0033383], geranylgeranyl diphosphate metabolic process [GO:0033385], farnesyl diphosphate metabolic process [GO:0045338], GO:0046490, lipid A metabolic process [GO:0046493], dimethylallyl diphosphate metabolic process [GO:0050993]